{
  "gene": "UniProtKB:Q8N841",
  "term_id": "GO:0001578",
  "term_label": "microtubule bundle formation",
  "gene_name": "Tubulin polyglutamylase TTLL6",
  "gene_symbol": "TTLL6"
}